{
  "gene_symbol": "ORC1",
  "gene_name": "Origin recognition complex subunit 1",
  "term_id": "GO:0006270",
  "gene": "UniProtKB:Q13415",
  "term_label": "DNA replication initiation"
}